{
  "term_id": "GO:0050650",
  "term_label": "chondroitin sulfate proteoglycan biosynthetic process",
  "gene_symbol": "XYLT1",
  "gene_name": "Xylosyltransferase 1",
  "gene": "UniProtKB:Q86Y38"
}